{
  "gene_symbol": "RDH11",
  "gene": "UniProtKB:Q8TC12",
  "term_label": "Unknown cellular component",
  "gene_name": "Retinol dehydrogenase 11",
  "term_id": "UNKNOWN:0003"
}